{
  "gene": "UniProtKB:Q8NGQ5",
  "gene_symbol": "OR9Q1",
  "term_id": "GO:0007608",
  "gene_name": "Olfactory receptor 9Q1",
  "term_label": "sensory perception of smell"
}